{
  "gene": "UniProtKB:P63096",
  "term_id": "GO:0003924",
  "gene_symbol": "GNAI1",
  "gene_name": "Guanine nucleotide-binding protein G(i) subunit alpha-1",
  "term_label": "GTPase activity"
}